{
  "term_id": "GO:0004321",
  "gene_symbol": "ACSM6",
  "term_label": "fatty-acyl-CoA synthase activity",
  "gene_name": "Acyl-coenzyme A synthetase ACSM6, mitochondrial",
  "gene": "UniProtKB:Q6P461"
}